{
  "gene_symbol": "NSD2",
  "term_id": "GO:0046975",
  "term_label": "histone H3K36 methyltransferase activity",
  "gene_name": "Histone-lysine N-methyltransferase NSD2",
  "gene": "UniProtKB:O96028"
}